{
  "term_id": "GO:0006357",
  "term_label": "regulation of transcription by RNA polymerase II",
  "gene_symbol": "ZNF420",
  "gene": "UniProtKB:Q8TAQ5",
  "gene_name": "Zinc finger protein 420"
}